{
  "term_label": "Unknown cellular component",
  "term_id": "UNKNOWN:0003",
  "gene_symbol": "FOXB2",
  "gene_name": "Forkhead box protein B2",
  "gene": "UniProtKB:Q5VYV0"
}